{
  "term_id": "GO:0034191",
  "gene": "UniProtKB:Q86UK0",
  "gene_name": "Glucosylceramide transporter ABCA12",
  "term_label": "apolipoprotein A-I receptor binding",
  "gene_symbol": "ABCA12"
}